{
  "gene_name": "Threonine--tRNA ligase 1, cytoplasmic",
  "gene": "UniProtKB:P26639",
  "term_id": "GO:0004829",
  "term_label": "threonine-tRNA ligase activity",
  "gene_symbol": "TARS1"
}